{
  "gene_symbol": "SMLR1",
  "term_label": "Unknown molecular function",
  "gene_name": "Small leucine-rich protein 1",
  "gene": "UniProtKB:H3BR10",
  "term_id": "UNKNOWN:0001"
}